sphingosine metabolic process [GO:0006670] (biological process) Definition: The chemical reactions and pathways involving sphingosine (sphing-4-enine), trans-D-erytho-2-amino-octadec-4-ene-1,3-diol, a long chain amino diol sphingoid base that occurs in most sphingolipids in animal tissues. Sources: GOC:ma, ISBN:0198506732 Also known as: (4E)-sphing-4-enine metabolic process, (4E)-sphing-4-enine metabolism, sphing-4-enine metabolic process, sphing-4-enine metabolism, sphingosine metabolism Relationships: is a type of diol metabolic process [GO:0034311]; is a type of sphingoid metabolic process [GO:0046519] Subtypes: sphingosine biosynthetic process [GO:0046512], GO:0051872